{
  "term_id": "UNKNOWN:0003",
  "term_label": "Unknown cellular component",
  "gene_symbol": "B3GALT5-AS1",
  "gene_name": "Putative uncharacterized protein B3GALT5-AS1",
  "gene": "UniProtKB:P59052"
}